{
  "gene": "UniProtKB:P80723",
  "gene_name": "Brain acid soluble protein 1",
  "term_id": "GO:0005634",
  "term_label": "nucleus",
  "gene_symbol": "BASP1"
}